traversing start control point of mitotic cell cycle [GO:0007089] (biological process) Sources: GOC:mtg_cell_cycle Definition: A cell cycle process by which a cell commits to entering S phase via a positive feedback mechanism between the regulation of transcription and G1 CDK activity. Relationships: is a type of positive regulation of G1/S transition of mitotic cell cycle [GO:1900087]